{
  "term_id": "UNKNOWN:0003",
  "gene_name": "Bublin coiled-coil protein",
  "term_label": "Unknown cellular component",
  "gene_symbol": "BBLN",
  "gene": "UniProtKB:Q9BUW7"
}